{
  "gene_name": "Homeobox protein DLX-1",
  "term_label": "regulation of transcription by RNA polymerase II",
  "term_id": "GO:0006357",
  "gene": "UniProtKB:P56177",
  "gene_symbol": "DLX1"
}